{
  "gene_symbol": "BRS3",
  "gene": "UniProtKB:P32247",
  "gene_name": "Bombesin receptor subtype-3",
  "term_label": "G protein-coupled receptor signaling pathway",
  "term_id": "GO:0007186"
}